long-chain-alcohol oxidase activity [GO:0046577] (molecular function) Also known as: fatty alcohol oxidase activity, long-chain fatty alcohol oxidase activity, fatty alcohol:oxygen oxidoreductase activity, long-chain fatty acid oxidase activity, long-chain-alcohol:oxygen oxidoreductase activity Sources: EC:1.1.3.20 Relationships: is a type of oxidoreductase activity, acting on the CH-OH group of donors, oxygen as acceptor [GO:0016899] Definition: Catalysis of the reaction: 2 long-chain alcohol + O2 = 2 long-chain aldehyde + 2 H2O.